COMA complex [GO:0000817] (CC) Definition: A kinetochore multiprotein complex that bridges the subunits that are in contact with centromeric DNA and the subunits bound to microtubules during kinetochore assembly. In yeast, consists of Ctf19p, Okp1p, Mcm21p, and Ame1p. References: PMID:14633972 Sources: GOC:se Also known as: Ctf19p-Okp1p-Mcm1p-Ame1p complex Relationships: is_a nuclear protein-containing complex [GO:0140513]; BFO_0000050 GO:0000228; is part of GO:0000776